stimulatory killer cell immunoglobulin-like receptor signaling pathway [GO:0002222] (biological process) Definition: The series of molecular signals initiated by a ligand binding to a killer cell immunoglobulin-like receptor capable of cellular activation. Sources: GOC:add, GO_REF:0000022, ISBN:0781735149 Also known as: stimulatory KIR signaling pathway, stimulatory killer cell immunoglobulin-like receptor signalling pathway Relationships: is a type of innate immune response activating cell surface receptor signaling pathway [GO:0002220]